{
  "term_id": "GO:0005634",
  "gene_name": "Mineralocorticoid receptor",
  "gene_symbol": "NR3C2",
  "term_label": "nucleus",
  "gene": "UniProtKB:P08235"
}